basal transcription machinery binding [GO:0001098] (molecular function) Definition: Binding to a component of the basal transcription machinery which is composed of the RNA polymerase core enzyme and the basal transcription factor(s), the minimal set of factors required for formation of the preinitiation complex (PIC) by the RNA polymerase. Sources: GOC:txnOH Relationships: is a type of protein binding [GO:0005515] Note: Note that the definition of basal, or general, transcription factors has typically been done at a small number of well characterized activator-independent promoters. At an activator-dependent promoter, one or more additional factors are generally required in addition to the basal factors. Subtypes: GO:0001099, bacterial-type RNA polymerase holo enzyme binding [GO:0001108]